menarche [GO:0042696] (biological process) References: PMID:16311040 Sources: GOC:curators Note: Note that this term should not be used for direct annotation. If you are trying to make an annotation to x phase, it is likely that the correct annotation is 'regulation of x/y phase transition' or to a process which occurs during the reported phase. To capture the phase when a specific location or process is observed, the phase term can be used in an annotation extension (PMID:24885854) applied to a cellular component term (with the relation exists_during) or a biological process term (with the relation happens_during). Definition: The beginning of the menstrual cycle; the first menstrual cycle in an individual. Relationships: is_a menstrual cycle phase [GO:0022601]